{
  "term_id": "GO:0035556",
  "gene_symbol": "STK38L",
  "gene": "UniProtKB:Q9Y2H1",
  "term_label": "intracellular signal transduction",
  "gene_name": "Serine_threonine-protein kinase 38-like"
}